2-hydroxy-1,4-benzoquinone reductase (NADH) activity [GO:0050625] (molecular function) Sources: RHEA:12428 Definition: Catalysis of the reaction: 2-hydroxy-1,4-benzoquinone + 2 H+ + NADH = benzene-1,2,4-triol + NAD+. Relationships: is_a oxidoreductase activity, acting on NAD(P)H, quinone or similar compound as acceptor [GO:0016655] Also known as: 2-hydroxy-1,4-benzoquinone reductase activity, 1,2,4-trihydroxybenzene:NAD oxidoreductase activity, 1,2,4-trihydroxybenzene:NAD+ oxidoreductase activity, 2-hydroxy-1,4-benzoquinone:NADH oxidoreductase activity, NADH:2-hydroxy-1,4-benzoquinone oxidoreductase activity, hydroxybenzoquinone reductase activity